{
  "gene": "UniProtKB:M0QZC1",
  "gene_symbol": "RNF225",
  "term_id": "GO:0016567",
  "term_label": "protein ubiquitination",
  "gene_name": "RING finger protein 225"
}